nuclear proteasome core complex [GO:0031601] (CC) Sources: GOC:mah Relationships: is a type of proteasome core complex [GO:0005839]; is a type of nuclear protein-containing complex [GO:0140513]; is part of nuclear proteasome complex [GO:0031595] Definition: The core complex of a proteasome located in the nucleus of a cell.